BH4 domain binding [GO:0051435] (MF) Definition: Binding to a BH4 protein domain, present in Bcl-2 family members. All anti-apoptotic proteins contain BH1 and BH2 domains; some also contain an additional N-terminal BH4 domain, which is almost never seen in pro-apoptotic proteins. Loss of the BH4 domain can diminish or abrogate anti-apoptotic function or even impart outright death-promoting properties to the protein. Relationships: is_a BH domain binding [GO:0051400] References: PMID:11048732, PMID:12133724, PMID:9020082, PMID:9704409 Sources: InterPro:IPR003093, Prosite:PS01260, Prosite:PS50063